protein homotrimerization [GO:0070207] (biological process) Sources: GOC:hjd Definition: The formation of a protein homotrimer, a macromolecular structure consisting of three noncovalently associated identical subunits. Relationships: is a type of protein homooligomerization [GO:0051260]; is a type of protein trimerization [GO:0070206] Also known as: protein homotrimer assembly, protein homotrimer biosynthesis, protein homotrimer biosynthetic process, protein homotrimer formation